{
  "gene_symbol": "POM121C",
  "term_id": "GO:0017056",
  "term_label": "structural constituent of nuclear pore",
  "gene_name": "Nuclear envelope pore membrane protein POM 121C",
  "gene": "UniProtKB:A8CG34"
}